{
  "gene_symbol": "SF3B3",
  "term_id": "GO:0005686",
  "term_label": "U2 snRNP",
  "gene_name": "Splicing factor 3B subunit 3",
  "gene": "UniProtKB:Q15393"
}